histamine N-methyltransferase activity [GO:0046539] (molecular function) Definition: Catalysis of the reaction: S-adenosyl-L-methionine(1+) + histamine = N(tau)-methylhistamine + S-adenosyl-L-homocysteine + H+. Sources: EC:2.1.1.8, RHEA:19301 Also known as: S-adenosyl-L-methionine:histamine N-tele-methyltransferase activity, S-adenosylmethionine-histamine N-methyltransferase activity, histamine 1-methyltransferase activity, histamine methyltransferase activity, histamine-methylating enzyme, imidazolemethyltransferase activity Relationships: is a type of N-methyltransferase activity [GO:0008170]; is_a GO:0008757